{
  "gene_name": "Protein FAM8A1",
  "gene": "UniProtKB:Q9UBU6",
  "term_id": "UNKNOWN:0002",
  "term_label": "Unknown biological process",
  "gene_symbol": "FAM8A1"
}